{
  "term_label": "endopeptidase activity",
  "gene": "UniProtKB:Q96T52",
  "gene_name": "Mitochondrial inner membrane protease subunit 2",
  "gene_symbol": "IMMP2L",
  "term_id": "GO:0004175"
}